{
  "gene_name": "Probable ATP-dependent RNA helicase DDX47",
  "gene_symbol": "DDX47",
  "term_label": "nucleus",
  "term_id": "GO:0005634",
  "gene": "UniProtKB:Q9H0S4"
}